{
  "term_label": "plasma membrane",
  "term_id": "GO:0005886",
  "gene_symbol": "MRGPRF",
  "gene_name": "Mas-related G-protein coupled receptor member F",
  "gene": "UniProtKB:Q96AM1"
}